{
  "gene": "UniProtKB:P55010",
  "gene_name": "Eukaryotic translation initiation factor 5",
  "term_id": "GO:0005092",
  "term_label": "GDP-dissociation inhibitor activity",
  "gene_symbol": "EIF5"
}